pi-body [GO:0071546] (cellular component) References: PMID:20011505 Sources: GOC:sp Definition: A P granule that contains the PIWIL2-TDRD1 module, a set of proteins that act in the primary piRNA pathway. The pi-body corresponds to the cementing material between mitochondria found in gonocytes. Relationships: is a type of P granule [GO:0043186] Also known as: intermitochondrial cement